{
  "gene": "UniProtKB:Q99685",
  "term_label": "monoacylglycerol lipase activity",
  "gene_name": "Monoglyceride lipase",
  "term_id": "GO:0047372",
  "gene_symbol": "MGLL"
}